{
  "term_id": "GO:0005654",
  "gene": "UniProtKB:O15355",
  "gene_symbol": "PPM1G",
  "gene_name": "Protein phosphatase 1G",
  "term_label": "nucleoplasm"
}